{
  "gene_name": "A-kinase anchor protein 2",
  "term_id": "UNKNOWN:0001",
  "gene_symbol": "AKAP2",
  "gene": "UniProtKB:Q9Y2D5",
  "term_label": "Unknown molecular function"
}